{
  "gene": "UniProtKB:Q9H5I5",
  "term_label": "cellular response to mechanical stimulus",
  "gene_name": "Piezo-type mechanosensitive ion channel component 2",
  "term_id": "GO:0071260",
  "gene_symbol": "PIEZO2"
}